{
  "gene_symbol": "KRTAP5-4",
  "term_label": "Unknown molecular function",
  "gene_name": "Keratin-associated protein 5-4",
  "gene": "UniProtKB:Q6L8H1",
  "term_id": "UNKNOWN:0001"
}